negative regulation of apoptotic process involved in development [GO:1904746] (biological process) Relationships: is a type of negative regulation of apoptotic process [GO:0043066]; is a type of negative regulation of developmental process [GO:0051093]; is a type of regulation of apoptotic process involved in development [GO:1904748]; negatively regulates GO:1902742 Subtypes: GO:0002868, GO:0045849, GO:1900212, negative regulation of apoptotic process involved in metanephric collecting duct development [GO:1900215], GO:1900218, negative regulation of apoptotic process involved in morphogenesis [GO:1902338] Definition: Any process that stops, prevents or reduces the frequency, rate or extent of apoptotic process involved in development. Note: U4PR86 in PMID:22801495 inferred from mutant phenotype References: PMID:22801495 Sources: GOC:TermGenie, GO_REF:0000058 Also known as: down regulation of apoptotic cell death involved in anatomical structure development, down regulation of apoptotic cell death involved in development of an anatomical structure, down regulation of apoptotic process involved in anatomical structure development, down regulation of apoptotic process involved in development, down regulation of apoptotic process involved in development of an anatomical structure, down regulation of apoptotic programmed cell death involved in anatomical structure development, down regulation of apoptotic programmed cell death involved in development of an anatomical structure, down regulation of programmed cell death by apoptosis involved in anatomical structure development, down regulation of programmed cell death by apoptosis involved in development of an anatomical structure, down-regulation of apoptotic cell death involved in anatomical structure development, down-regulation of apoptotic cell death involved in development of an anatomical structure, down-regulation of apoptotic process involved in anatomical structure development, down-regulation of apoptotic process involved in development, down-regulation of apoptotic process involved in development of an anatomical structure, down-regulation of apoptotic programmed cell death involved in anatomical structure development, down-regulation of apoptotic programmed cell death involved in development of an anatomical structure, down-regulation of programmed cell death by apoptosis involved in anatomical structure development, down-regulation of programmed cell death by apoptosis involved in development of an anatomical structure, downregulation of apoptotic cell death involved in anatomical structure development, downregulation of apoptotic cell death involved in development of an anatomical structure, downregulation of apoptotic process involved in anatomical structure development, downregulation of apoptotic process involved in development, downregulation of apoptotic process involved in development of an anatomical structure, downregulation of apoptotic programmed cell death involved in anatomical structure development, downregulation of apoptotic programmed cell death involved in development of an anatomical structure, downregulation of programmed cell death by apoptosis involved in anatomical structure development, downregulation of programmed cell death by apoptosis involved in development of an anatomical structure, negative regulation of apoptotic cell death involved in anatomical structure development, negative regulation of apoptotic cell death involved in development of an anatomical structure, negative regulation of apoptotic process involved in anatomical structure development, negative regulation of apoptotic process involved in development of an anatomical structure, negative regulation of apoptotic programmed cell death involved in anatomical structure development, negative regulation of apoptotic programmed cell death involved in development of an anatomical structure, negative regulation of programmed cell death by apoptosis involved in anatomical structure development, negative regulation of programmed cell death by apoptosis involved in development of an anatomical structure, down regulation of activation of apoptosis involved in anatomical structure development, down regulation of activation of apoptosis involved in development of an anatomical structure, down regulation of apoptosis involved in anatomical structure development, down regulation of apoptosis involved in development of an anatomical structure, down regulation of apoptosis signaling involved in anatomical structure development, down regulation of apoptosis signaling involved in development of an anatomical structure, down regulation of apoptotic program involved in anatomical structure development, down regulation of apoptotic program involved in development of an anatomical structure, down regulation of type I programmed cell death involved in anatomical structure development, down regulation of type I programmed cell death involved in development of an anatomical structure, down-regulation of activation of apoptosis involved in anatomical structure development, down-regulation of activation of apoptosis involved in development of an anatomical structure, down-regulation of apoptosis involved in anatomical structure development, down-regulation of apoptosis involved in development of an anatomical structure, down-regulation of apoptosis signaling involved in anatomical structure development, down-regulation of apoptosis signaling involved in development of an anatomical structure, down-regulation of apoptotic program involved in anatomical structure development, down-regulation of apoptotic program involved in development of an anatomical structure, down-regulation of type I programmed cell death involved in anatomical structure development, down-regulation of type I programmed cell death involved in development of an anatomical structure, downregulation of activation of apoptosis involved in anatomical structure development, downregulation of activation of apoptosis involved in development of an anatomical structure, downregulation of apoptosis involved in anatomical structure development, downregulation of apoptosis involved in development of an anatomical structure, downregulation of apoptosis signaling involved in anatomical structure development, downregulation of apoptosis signaling involved in development of an anatomical structure, downregulation of apoptotic program involved in anatomical structure development, downregulation of apoptotic program involved in development of an anatomical structure, downregulation of type I programmed cell death involved in anatomical structure development, downregulation of type I programmed cell death involved in development of an anatomical structure, inhibition of activation of apoptosis involved in anatomical structure development, inhibition of activation of apoptosis involved in development of an anatomical structure, inhibition of apoptosis involved in anatomical structure development, inhibition of apoptosis involved in development of an anatomical structure, inhibition of apoptosis signaling involved in anatomical structure development, inhibition of apoptosis signaling involved in development of an anatomical structure, inhibition of apoptotic cell death involved in anatomical structure development, inhibition of apoptotic cell death involved in development of an anatomical structure, inhibition of apoptotic process involved in anatomical structure development, inhibition of apoptotic process involved in development, inhibition of apoptotic process involved in development of an anatomical structure, inhibition of apoptotic program involved in anatomical structure development, inhibition of apoptotic program involved in development of an anatomical structure, inhibition of apoptotic programmed cell death involved in anatomical structure development, inhibition of apoptotic programmed cell death involved in development of an anatomical structure, inhibition of programmed cell death by apoptosis involved in anatomical structure development, inhibition of programmed cell death by apoptosis involved in development of an anatomical structure, inhibition of type I programmed cell death involved in anatomical structure development, inhibition of type I programmed cell death involved in development of an anatomical structure, negative regulation of activation of apoptosis involved in anatomical structure development, negative regulation of activation of apoptosis involved in development of an anatomical structure, negative regulation of apoptosis involved in anatomical structure development, negative regulation of apoptosis involved in development of an anatomical structure, negative regulation of apoptosis signaling involved in anatomical structure development, negative regulation of apoptosis signaling involved in development of an anatomical structure, negative regulation of apoptotic program involved in anatomical structure development, negative regulation of apoptotic program involved in development of an anatomical structure, negative regulation of type I programmed cell death involved in anatomical structure development, negative regulation of type I programmed cell death involved in development of an anatomical structure, down regulation of apoptosis activator activity involved in anatomical structure development, down regulation of apoptosis activator activity involved in development of an anatomical structure, down regulation of commitment to apoptosis involved in anatomical structure development, down regulation of commitment to apoptosis involved in development of an anatomical structure, down regulation of induction of apoptosis by p53 involved in anatomical structure development, down regulation of induction of apoptosis by p53 involved in development of an anatomical structure, down regulation of induction of apoptosis involved in anatomical structure development, down regulation of induction of apoptosis involved in development of an anatomical structure, down regulation of signaling (initiator) caspase activity involved in anatomical structure development, down regulation of signaling (initiator) caspase activity involved in development of an anatomical structure, down-regulation of apoptosis activator activity involved in anatomical structure development, down-regulation of apoptosis activator activity involved in development of an anatomical structure, down-regulation of commitment to apoptosis involved in anatomical structure development, down-regulation of commitment to apoptosis involved in development of an anatomical structure, down-regulation of induction of apoptosis by p53 involved in anatomical structure development, down-regulation of induction of apoptosis by p53 involved in development of an anatomical structure, down-regulation of induction of apoptosis involved in anatomical structure development, down-regulation of induction of apoptosis involved in development of an anatomical structure, down-regulation of signaling (initiator) caspase activity involved in anatomical structure development, down-regulation of signaling (initiator) caspase activity involved in development of an anatomical structure, downregulation of apoptosis activator activity involved in anatomical structure development, downregulation of apoptosis activator activity involved in development of an anatomical structure, downregulation of commitment to apoptosis involved in anatomical structure development, downregulation of commitment to apoptosis involved in development of an anatomical structure, downregulation of induction of apoptosis by p53 involved in anatomical structure development, downregulation of induction of apoptosis by p53 involved in development of an anatomical structure, downregulation of induction of apoptosis involved in anatomical structure development, downregulation of induction of apoptosis involved in development of an anatomical structure, downregulation of signaling (initiator) caspase activity involved in anatomical structure development, downregulation of signaling (initiator) caspase activity involved in development of an anatomical structure, inhibition of apoptosis activator activity involved in anatomical structure development, inhibition of apoptosis activator activity involved in development of an anatomical structure, inhibition of commitment to apoptosis involved in anatomical structure development, inhibition of commitment to apoptosis involved in development of an anatomical structure, inhibition of induction of apoptosis by p53 involved in anatomical structure development, inhibition of induction of apoptosis by p53 involved in development of an anatomical structure, inhibition of induction of apoptosis involved in anatomical structure development, inhibition of induction of apoptosis involved in development of an anatomical structure, inhibition of signaling (initiator) caspase activity involved in anatomical structure development, inhibition of signaling (initiator) caspase activity involved in development of an anatomical structure, negative regulation of apoptosis activator activity involved in anatomical structure development, negative regulation of apoptosis activator activity involved in development of an anatomical structure, negative regulation of commitment to apoptosis involved in anatomical structure development, negative regulation of commitment to apoptosis involved in development of an anatomical structure, negative regulation of induction of apoptosis by p53 involved in anatomical structure development, negative regulation of induction of apoptosis by p53 involved in development of an anatomical structure, negative regulation of induction of apoptosis involved in anatomical structure development, negative regulation of induction of apoptosis involved in development of an anatomical structure, negative regulation of signaling (initiator) caspase activity involved in anatomical structure development, negative regulation of signaling (initiator) caspase activity involved in development of an anatomical structure